{
  "gene_name": "Bublin coiled-coil protein",
  "term_id": "UNKNOWN:0001",
  "gene": "UniProtKB:Q9BUW7",
  "gene_symbol": "BBLN",
  "term_label": "Unknown molecular function"
}